{
  "gene_name": "Membrane protein FAM174A",
  "term_id": "UNKNOWN:0001",
  "term_label": "Unknown molecular function",
  "gene": "UniProtKB:Q8TBP5",
  "gene_symbol": "FAM174A"
}